{
  "term_id": "UNKNOWN:0001",
  "term_label": "Unknown molecular function",
  "gene_symbol": "C1orf100",
  "gene": "UniProtKB:Q5SVJ3",
  "gene_name": "Uncharacterized protein C1orf100"
}